{
  "gene_name": "Cullin-3",
  "term_id": "GO:0031463",
  "term_label": "Cul3-RING ubiquitin ligase complex",
  "gene_symbol": "CUL3",
  "gene": "UniProtKB:Q13618"
}